{
  "gene_symbol": "L3MBTL3",
  "gene_name": "Lethal(3)malignant brain tumor-like protein 3",
  "term_label": "nucleus",
  "gene": "UniProtKB:Q96JM7",
  "term_id": "GO:0005634"
}